{
  "gene_name": "Histone deacetylase 3",
  "gene_symbol": "HDAC3",
  "gene": "UniProtKB:O15379",
  "term_id": "GO:0040029",
  "term_label": "epigenetic regulation of gene expression"
}